{
  "term_label": "apoptotic process involved in development",
  "gene": "UniProtKB:Q5GH72",
  "gene_name": "XK-related protein 7",
  "term_id": "GO:1902742",
  "gene_symbol": "XKR7"
}